{
  "gene_symbol": "ABCD4",
  "term_id": "GO:0005778",
  "gene_name": "Lysosomal cobalamin transporter ABCD4",
  "gene": "UniProtKB:O14678",
  "term_label": "peroxisomal membrane"
}